{
  "gene_symbol": "KIAA0040",
  "gene": "UniProtKB:Q15053",
  "gene_name": "Uncharacterized protein KIAA0040",
  "term_id": "UNKNOWN:0002",
  "term_label": "Unknown biological process"
}